{
  "term_label": "Unknown molecular function",
  "gene_name": "Uncharacterized protein C3orf84",
  "gene": "UniProtKB:H3BNL1",
  "term_id": "UNKNOWN:0001",
  "gene_symbol": "C3orf84"
}